collagen type XXVIII trimer [GO:1990326] (cellular component) References: PMID:17876790 Definition: A collagen homotrimer of alpha1(XXVIII) chains. Relationships: is a type of von-Willerbrand-factor-A-domain-rich collagen trimer [GO:0140158]; is part of GO:0140143